{
  "term_id": "GO:0005739",
  "gene_symbol": "TMEM126B",
  "term_label": "mitochondrion",
  "gene": "UniProtKB:Q8IUX1",
  "gene_name": "Complex I assembly factor TMEM126B, mitochondrial"
}